positive regulation of microtubule depolymerization [GO:0031117] (biological process) Definition: Any process that activates or increases the frequency, rate or extent of microtubule depolymerization. Also known as: microtubule destabilization, positive regulation of microtubule disassembly, up regulation of microtubule depolymerization, up-regulation of microtubule depolymerization, upregulation of microtubule depolymerization, activation of microtubule depolymerization, positive regulation of microtubule catastrophe, stimulation of microtubule depolymerization Sources: GOC:mah Relationships: is a type of positive regulation of microtubule polymerization or depolymerization [GO:0031112]; is a type of regulation of microtubule depolymerization [GO:0031114]; is a type of positive regulation of protein depolymerization [GO:1901881]; is a type of GO:1902905; positively regulates microtubule depolymerization [GO:0007019]